{
  "gene": "UniProtKB:Q6UUV7",
  "term_label": "cellular response to cAMP",
  "gene_name": "CREB-regulated transcription coactivator 3",
  "gene_symbol": "CRTC3",
  "term_id": "GO:0071320"
}